{
  "gene_symbol": "MKS1",
  "gene_name": "Tectonic-like complex member MKS1",
  "term_label": "MKS complex",
  "gene": "UniProtKB:Q9NXB0",
  "term_id": "GO:0036038"
}